{
  "gene": "UniProtKB:Q9NZR1",
  "gene_name": "Tropomodulin-2",
  "term_label": "myofibril assembly",
  "gene_symbol": "TMOD2",
  "term_id": "GO:0030239"
}